{
  "gene_name": "Pentatricopeptide repeat-containing protein 1, mitochondrial",
  "term_label": "tRNA 3'-end processing",
  "gene": "UniProtKB:O75127",
  "gene_symbol": "PTCD1",
  "term_id": "GO:0042780"
}